{
  "gene": "UniProtKB:P58550",
  "term_label": "sodium channel regulator activity",
  "gene_name": "Putative FXYD domain-containing ion transport regulator 8",
  "gene_symbol": "FXYD6P3",
  "term_id": "GO:0017080"
}